{
  "gene": "UniProtKB:Q49AN0",
  "term_label": "circadian regulation of gene expression",
  "term_id": "GO:0032922",
  "gene_name": "Cryptochrome-2",
  "gene_symbol": "CRY2"
}